positive regulation of pancreatic juice secretion [GO:0090187] (biological process) Sources: GOC:BHF, GOC:dph, GOC:tb Relationships: is a type of GO:0051047; is_a positive regulation of digestive system process [GO:0060456]; is_a GO:0090186; positively regulates pancreatic juice secretion [GO:0030157] Definition: Any process that increases the rate, frequency or extent of pancreatic juice secretion, the regulated release of pancreatic juice by the exocrine pancreas into the upper part of the intestine.